{
  "gene_symbol": "RAB7B",
  "gene": "UniProtKB:Q96AH8",
  "term_label": "endosome to lysosome transport",
  "gene_name": "Ras-related protein Rab-7b",
  "term_id": "GO:0008333"
}